{
  "gene_symbol": "NPEPL1",
  "term_id": "GO:0006508",
  "gene": "UniProtKB:Q8NDH3",
  "term_label": "proteolysis",
  "gene_name": "Probable aminopeptidase NPEPL1"
}